{
  "term_id": "GO:0008009",
  "term_label": "chemokine activity",
  "gene_symbol": "XCL2",
  "gene_name": "Cytokine SCM-1 beta",
  "gene": "UniProtKB:Q9UBD3"
}